{
  "term_id": "GO:0005737",
  "term_label": "cytoplasm",
  "gene_name": "Serine_threonine-protein kinase TNNI3K",
  "gene_symbol": "TNNI3K",
  "gene": "UniProtKB:Q59H18"
}